{
  "gene_symbol": "CFAP91",
  "term_id": "UNKNOWN:0001",
  "gene": "UniProtKB:Q7Z4T9",
  "gene_name": "Cilia- and flagella-associated protein 91",
  "term_label": "Unknown molecular function"
}